(iso)eugenol O-methyltransferase activity [GO:0050630] (molecular function) Also known as: isoeugenol O-methyltransferase activity, S-adenosyl-L-methionine:isoeugenol O-methyltransferase activity Sources: RHEA:17081 Definition: Catalysis of the reaction: (E)-isoeugenol + S-adenosyl-L-methionine = (E)-isomethyleugenol + H+ + S-adenosyl-L-homocysteine. Relationships: is a type of O-methyltransferase activity [GO:0008171]